{
  "gene": "UniProtKB:A0A075B6Y0",
  "term_id": "UNKNOWN:0002",
  "gene_name": "T cell receptor alpha joining 49 (Fragment)",
  "term_label": "Unknown biological process",
  "gene_symbol": "TRAJ49"
}